placenta development [GO:0001890] (biological process) Definition: The process whose specific outcome is the progression of the placenta over time, from its formation to the mature structure. The placenta is an organ of metabolic interchange between fetus and mother, partly of embryonic origin and partly of maternal origin. Sources: GOC:add, ISBN:068340007X Also known as: placental development, placentation Relationships: is a type of GO:0048513